cell surface adhesin-mediated gliding motility [GO:0071980] (biological process) Definition: Cell gliding that results from the actions of cell surface adhesin proteins that are propelled by membrane motor proteins. Relationships: is a type of GO:0071976 References: PMID:18461074